{
  "gene_symbol": "SETD3",
  "gene": "UniProtKB:Q86TU7",
  "term_id": "GO:0070472",
  "term_label": "regulation of uterine smooth muscle contraction",
  "gene_name": "Actin-histidine N-methyltransferase"
}